{
  "gene": "UniProtKB:Q9Y496",
  "term_label": "anterograde axonal transport",
  "gene_symbol": "KIF3A",
  "term_id": "GO:0008089",
  "gene_name": "Kinesin-like protein KIF3A"
}